{
  "gene_name": "Fibroblast growth factor 10",
  "term_label": "type 2 fibroblast growth factor receptor binding",
  "gene": "UniProtKB:O15520",
  "term_id": "GO:0005111",
  "gene_symbol": "FGF10"
}